{
  "gene_name": "Sulfite oxidase, mitochondrial",
  "term_id": "GO:0043546",
  "gene": "UniProtKB:P51687",
  "gene_symbol": "SUOX",
  "term_label": "molybdopterin cofactor binding"
}